{
  "gene_name": "Deleted in azoospermia protein 1",
  "term_id": "GO:0005737",
  "term_label": "cytoplasm",
  "gene_symbol": "DAZ1",
  "gene": "UniProtKB:Q9NQZ3"
}